{
  "gene_name": "NKG2-E type II integral membrane protein",
  "term_label": "activating MHC class Ib receptor activity",
  "term_id": "GO:0062081",
  "gene_symbol": "KLRC3",
  "gene": "UniProtKB:Q07444"
}